{
  "term_label": "regulation of organ growth",
  "gene_name": "Serine_threonine-protein kinase LATS2",
  "gene": "UniProtKB:Q9NRM7",
  "gene_symbol": "LATS2",
  "term_id": "GO:0046620"
}